nicotinate-nucleotide-dimethylbenzimidazole phosphoribosyltransferase activity [GO:0008939] (molecular function) Sources: EC:2.4.2.21, RHEA:11196 Also known as: CobT, N(1)-alpha-phosphoribosyltransferase activity, N1-alpha-phosphoribosyltransferase activity, nicotinate mononucleotide (NaMN):5,6-dimethylbenzimidazole phosphoribosyltransferase activity, nicotinate mononucleotide-dimethylbenzimidazole phosphoribosyltransferase activity, nicotinate ribonucleotide:benzimidazole (adenine) phosphoribosyltransferase activity, nicotinate-nucleotide:5,6-dimethylbenzimidazole phospho-D-ribosyltransferase activity, nicotinate-nucleotide:dimethylbenzimidazole phospho-D-ribosyltransferase activity Definition: Catalysis of the reaction: 5,6-dimethylbenzimidazole + nicotinate D-ribonucleotide = alpha-ribazole 5'-phosphate + H+ + nicotinate. Relationships: is a type of GO:0016763